{
  "gene_name": "Plexin-B1",
  "term_id": "GO:0030334",
  "gene": "UniProtKB:O43157",
  "term_label": "regulation of cell migration",
  "gene_symbol": "PLXNB1"
}